{
  "term_label": "structural constituent of cytoskeleton",
  "gene_symbol": "TUBB3",
  "gene": "UniProtKB:Q13509",
  "gene_name": "Tubulin beta-3 chain",
  "term_id": "GO:0005200"
}